regulation of heme biosynthetic process [GO:0070453] (biological process) Definition: Any process that modulates the frequency, rate or extent of the chemical reactions and pathways resulting in the formation of heme. Subtypes: GO:0070454, positive regulation of heme biosynthetic process [GO:0070455] Also known as: regulation of haem biosynthesis, regulation of haem biosynthetic process, regulation of heme anabolism, regulation of heme biosynthesis, regulation of heme formation, regulation of heme synthesis Sources: GOC:mah Relationships: is a type of regulation of tetrapyrrole biosynthetic process [GO:1901463]; regulates heme biosynthetic process [GO:0006783]